phospholipase C inhibitor activity [GO:0160186] (molecular function) References: PMID:28130414 Relationships: is a type of phospholipase inhibitor activity [GO:0004859]; negatively regulates phospholipase C activity [GO:0004629] Definition: Binds to and stops, prevents or reduces the activity of the enzyme phospholipase C.